{
  "gene_name": "Hemoglobin subunit gamma-2",
  "term_label": "erythrocyte development",
  "gene": "UniProtKB:P69892",
  "gene_symbol": "HBG2",
  "term_id": "GO:0048821"
}